ribose 1,5-bisphosphate isomerase activity [GO:0043917] (molecular function) Definition: Catalysis of the reaction: alpha-D-ribose 1,5-bisphosphate = D-ribulose 1,5-bisphosphate. Sources: RHEA:32243 Also known as: ribose-1,5-bisphosphate isomerase activity Relationships: is_a intramolecular oxidoreductase activity, interconverting aldoses and ketoses [GO:0016861]